macropinosomal membrane permeabilization involved in viral entry into host cell [GO:0075504] (biological process) Definition: Induction of macropinosome membrane permeabilization triggered by an interaction between the host membrane and a membrane-penetration protein associated with the capsid. Occurs after internalization of the virus in a macropinosome, and results in release of the viral contents from the macropinosome into the host cell cytoplasm. Sources: GOC:bf, GOC:jl Also known as: viral entry into host cell via macropinocytosis followed by macropinosomal membrane permeabilization Relationships: is a type of GO:0039665